cell wall-bounded periplasmic space [GO:0030287] (CC) Also known as: cell wall bounded periplasmic space, cell wall-enclosed periplasmic space, IWZ, inner wall zone Sources: GOC:mlg, GOC:mtg_sensu Relationships: is a type of periplasmic space [GO:0042597] Definition: The region between the plasma membrane and the cell wall in organisms lacking an outer cell membrane such as yeast and Gram positive bacteria. The region is thinner than the equivalent in Gram negative bacteria.